{
  "term_label": "cilium-dependent cell motility",
  "gene": "UniProtKB:Q9NVR5",
  "gene_name": "Protein kintoun",
  "gene_symbol": "DNAAF2",
  "term_id": "GO:0060285"
}